kynurenine-oxoglutarate transaminase activity [GO:0016212] (molecular function) Sources: EC:2.6.1.7 Relationships: is a type of transaminase activity [GO:0008483] Definition: Catalysis of the reaction: 2-oxoglutarate + L-kynurenine = H2O + kynurenate + L-glutamate. The product 4-(2-aminophenyl)-2,4-dioxobutanoate is converted into kynurenate by a spontaneous reaction. Also acts on 3-hydroxykynurenine to form xanthurenate. Also known as: kynurenine aminotransferase activity, kynurenine-oxoglutarate aminotransferase activity, L-kynurenine aminotransferase activity, L-kynurenine:2-oxoglutarate aminotransferase activity, kynurenine 2-oxoglutarate transaminase activity, kynurenine transaminase (cyclizing), kynurenine--oxoglutarate aminotransferase activity